{
  "gene": "UniProtKB:Q08AN1",
  "term_id": "GO:0000981",
  "term_label": "DNA-binding transcription factor activity, RNA polymerase II-specific",
  "gene_name": "Zinc finger protein 616",
  "gene_symbol": "ZNF616"
}